{
  "gene": "UniProtKB:Q9H1Y3",
  "term_id": "GO:0008020",
  "gene_name": "Opsin-3",
  "term_label": "G protein-coupled photoreceptor activity",
  "gene_symbol": "OPN3"
}